{
  "gene_name": "Testis-specific Y-encoded-like protein 6",
  "gene_symbol": "TSPYL6",
  "term_id": "GO:0005634",
  "term_label": "nucleus",
  "gene": "UniProtKB:Q8N831"
}